{
  "gene_symbol": "MORC4",
  "term_id": "GO:0005634",
  "gene": "UniProtKB:Q8TE76",
  "gene_name": "MORC family CW-type zinc finger protein 4",
  "term_label": "nucleus"
}